{
  "gene": "UniProtKB:O75173",
  "gene_name": "A disintegrin and metalloproteinase with thrombospondin motifs 4",
  "gene_symbol": "ADAMTS4",
  "term_label": "extracellular matrix organization",
  "term_id": "GO:0030198"
}